{
  "term_label": "cell morphogenesis",
  "term_id": "GO:0000902",
  "gene_name": "Cadherin-12",
  "gene": "UniProtKB:P55289",
  "gene_symbol": "CDH12"
}